{
  "gene": "UniProtKB:Q15155",
  "term_id": "GO:0005789",
  "gene_symbol": "NOMO1",
  "term_label": "endoplasmic reticulum membrane",
  "gene_name": "BOS complex subunit NOMO1"
}